{
  "term_id": "GO:0019915",
  "term_label": "lipid storage",
  "gene_name": "Seipin",
  "gene": "UniProtKB:Q96G97",
  "gene_symbol": "BSCL2"
}